sensory perception of sour taste [GO:0050915] (biological process) Definition: The series of events required to receive a sour taste stimulus, convert it to a molecular signal, and recognize and characterize the signal. This is a neurological process. Relationships: is a type of sensory perception of taste [GO:0050909] Also known as: sour taste perception Sources: GOC:ai